{
  "term_id": "GO:0005634",
  "term_label": "nucleus",
  "gene": "UniProtKB:Q8TF20",
  "gene_name": "Zinc finger protein 721",
  "gene_symbol": "ZNF721"
}